{
  "gene_name": "Membrane-associated phosphatidylinositol transfer protein 1",
  "term_id": "GO:0031210",
  "term_label": "phosphatidylcholine binding",
  "gene": "UniProtKB:O00562",
  "gene_symbol": "PITPNM1"
}